embryonic organ development [GO:0048568] (biological process) Definition: Development, taking place during the embryonic phase, of a tissue or tissues that work together to perform a specific function or functions. Development pertains to the process whose specific outcome is the progression of a structure over time, from its formation to the mature structure. Organs are commonly observed as visibly distinct structures, but may also exist as loosely associated clusters of cells that work together to perform a specific function or functions. Subtypes: embryonic placenta development [GO:0001892], notochord development [GO:0030903], embryonic camera-type eye development [GO:0031076], embryonic hemopoiesis [GO:0035162], embryonic digestive tract development [GO:0048566], GO:0055016, labyrinthine layer blood vessel development [GO:0060716], embryonic lung development [GO:1990401], embryonic liver development [GO:1990402], GO:1990403 Sources: GOC:jid Also known as: embryonic organogenesis Relationships: is a type of GO:0048513; is part of embryo development [GO:0009790]